{
  "term_label": "Unknown molecular function",
  "gene": "UniProtKB:Q6ZR08",
  "gene_symbol": "DNAH12",
  "gene_name": "Dynein axonemal heavy chain 12",
  "term_id": "UNKNOWN:0001"
}